aryl-alcohol dehydrogenase (NADP+) activity [GO:0047681] (molecular function) Relationships: is a type of oxidoreductase activity, acting on the CH-OH group of donors, NAD or NADP as acceptor [GO:0016616] Definition: Catalysis of the reaction: an aromatic alcohol + NADP+ = an aromatic aldehyde + NADPH. Sources: EC:1.1.1.91, MetaCyc:ARYL-ALCOHOL-DEHYDROGENASE-NADP+-RXN Also known as: NADPH-linked benzaldehyde reductase activity, aryl alcohol dehydrogenase (nicotinamide adenine dinucleotide phosphate), aryl-alcohol:NADP+ oxidoreductase activity